{
  "term_label": "Golgi apparatus",
  "gene_symbol": "CEP83",
  "gene_name": "Centrosomal protein of 83 kDa",
  "gene": "UniProtKB:Q9Y592",
  "term_id": "GO:0005794"
}